{
  "term_id": "GO:0006457",
  "term_label": "protein folding",
  "gene": "UniProtKB:Q14554",
  "gene_symbol": "PDIA5",
  "gene_name": "Protein disulfide-isomerase A5"
}